regulation of multicellular organismal development [GO:2000026] (biological process) Subtypes: regulation of eclosion [GO:0007563], GO:0007564, regulation of epithelial cell differentiation [GO:0030856], regulation of skeletal muscle tissue regeneration [GO:0043416], GO:0045691, regulation of embryonic development [GO:0045995], regulation of post-embryonic development [GO:0048580], GO:0051797, regulation of nervous system development [GO:0051960], regulation of heart growth [GO:0060420], positive regulation of mammary placode formation by mesenchymal-epithelial signaling [GO:0060617], positive regulation of salivary gland formation by mesenchymal-epithelial signaling [GO:0060639], regulation of cartilage development [GO:0061035], regulation of biomineral tissue development [GO:0070167], regulation of metaxylem development [GO:0090060], regulation of vasculature development [GO:1901342], regulation of bone development [GO:1903010], regulation of lactation [GO:1903487], regulation of hemopoiesis [GO:1903706], GO:1905276, regulation of female gonad development [GO:2000194] Definition: Any process that modulates the frequency, rate or extent of multicellular organismal development. Sources: GOC:obol Relationships: is a type of regulation of developmental process [GO:0050793]; is a type of regulation of multicellular organismal process [GO:0051239]; regulates multicellular organism development [GO:0007275]